mitochondrial ATP transmembrane transport [GO:1990544] (BP) Relationships: is a type of GO:0015867; is a type of GO:0072530; is a type of GO:1901679 Definition: The process in which ATP is transported across a mitochondrial membrane, into or out of the mitochondrion. References: PMID:18485069